{
  "gene": "UniProtKB:A1E959",
  "gene_symbol": "ODAM",
  "term_id": "GO:0005737",
  "term_label": "cytoplasm",
  "gene_name": "Odontogenic ameloblast-associated protein"
}